{
  "gene": "UniProtKB:Q71UI9",
  "gene_symbol": "H2AZ2",
  "gene_name": "Histone H2A.V",
  "term_id": "GO:0030527",
  "term_label": "structural constituent of chromatin"
}